{
  "term_id": "GO:0005615",
  "gene_symbol": "EPX",
  "gene": "UniProtKB:P11678",
  "gene_name": "Eosinophil peroxidase",
  "term_label": "extracellular space"
}